{
  "gene": "UniProtKB:Q8WZA0",
  "term_label": "Unknown molecular function",
  "term_id": "UNKNOWN:0001",
  "gene_symbol": "LZIC",
  "gene_name": "Protein LZIC"
}